cobalt-precorrin-5B C1-methyltransferase activity [GO:0043780] (molecular function) Sources: MetaCyc:RXN-8764 Also known as: cobalt-precorrin 5B C1-methyltransferase activity Definition: Catalysis of the reaction: cobalt-precorrin 5B + S-adenosylmethionine = S-adenosylhomocysteine + cobalt-precorrin 6A. Relationships: is a type of GO:0008168